{
  "gene_symbol": "D2HGDH",
  "term_label": "Unknown biological process",
  "gene_name": "D-2-hydroxyglutarate dehydrogenase, mitochondrial",
  "gene": "UniProtKB:Q8N465",
  "term_id": "UNKNOWN:0002"
}